{
  "gene_name": "Ferritin light chain",
  "term_label": "Unknown biological process",
  "gene_symbol": "FTL",
  "gene": "UniProtKB:P02792",
  "term_id": "UNKNOWN:0002"
}